{
  "term_id": "UNKNOWN:0003",
  "gene_symbol": "KRTAP4-3",
  "gene_name": "Keratin-associated protein 4-3",
  "gene": "UniProtKB:Q9BYR4",
  "term_label": "Unknown cellular component"
}